negative regulation of chemotaxis [GO:0050922] (biological process) Also known as: down regulation of chemotaxis, down-regulation of chemotaxis, downregulation of chemotaxis, inhibition of chemotaxis Definition: Any process that stops, prevents, or reduces the frequency, rate or extent of the directed movement of a motile cell or organism in response to a specific chemical concentration gradient. Subtypes: negative regulation of leukocyte chemotaxis [GO:0002689], negative regulation of axon extension involved in axon guidance [GO:0048843], negative regulation of negative chemotaxis [GO:0050925], negative regulation of positive chemotaxis [GO:0050928], negative regulation of smooth muscle cell chemotaxis [GO:0071672], negative regulation of chemokine activity [GO:1900137], negative regulation of axon guidance [GO:1902668], negative regulation of Schwann cell chemotaxis [GO:1904267], negative regulation of chemotaxis to arachidonate [GO:1904553], negative regulation of cell chemotaxis to fibroblast growth factor [GO:1904848], GO:1904858, negative regulation of fibroblast chemotaxis [GO:1905211], GO:2000459, negative regulation of endothelial cell chemotaxis [GO:2001027], negative regulation of muscle cell chemotaxis toward tendon cell [GO:2001282] Sources: GOC:ai Relationships: is_a negative regulation of response to external stimulus [GO:0032102]; is a type of negative regulation of locomotion [GO:0040013]; is a type of regulation of chemotaxis [GO:0050920]; RO_0002212 chemotaxis [GO:0006935]